{
  "term_id": "UNKNOWN:0001",
  "gene_symbol": "FIZ1",
  "term_label": "Unknown molecular function",
  "gene": "UniProtKB:Q96SL8",
  "gene_name": "Flt3-interacting zinc finger protein 1"
}